{
  "term_label": "Unknown cellular component",
  "gene_symbol": "NACC2",
  "term_id": "UNKNOWN:0003",
  "gene": "UniProtKB:Q96BF6",
  "gene_name": "Nucleus accumbens-associated protein 2"
}